positive regulation of hyaluranon cable assembly [GO:1900106] (biological process) Relationships: is a type of positive regulation of cellular component biogenesis [GO:0044089]; is a type of GO:0051130; is a type of regulation of hyaluranon cable assembly [GO:1900104]; positively regulates hyaluranon cable assembly [GO:0036118] Also known as: activation of HA cable assembly, positive regulation of HA cable assembly, up regulation of HA cable assembly, up regulation of hyaluranon cable assembly, up-regulation of HA cable assembly, up-regulation of hyaluranon cable assembly, upregulation of HA cable assembly, upregulation of hyaluranon cable assembly, activation of hyaluranon cable assembly Sources: GOC:TermGenie, GOC:yaf Definition: Any process that activates or increases the frequency, rate or extent of hyaluranon cable assembly.